{
  "gene": "UniProtKB:P15153",
  "gene_name": "Ras-related C3 botulinum toxin substrate 2",
  "gene_symbol": "RAC2",
  "term_label": "GTP binding",
  "term_id": "GO:0005525"
}